{
  "gene": "UniProtKB:O75093",
  "term_id": "GO:0007411",
  "gene_symbol": "SLIT1",
  "gene_name": "Slit homolog 1 protein",
  "term_label": "axon guidance"
}